{
  "term_id": "GO:0005886",
  "gene_symbol": "RXFP1",
  "term_label": "plasma membrane",
  "gene_name": "Relaxin receptor 1",
  "gene": "UniProtKB:Q9HBX9"
}